{
  "gene_name": "Protein FAM222A",
  "term_id": "UNKNOWN:0002",
  "gene_symbol": "FAM222A",
  "term_label": "Unknown biological process",
  "gene": "UniProtKB:Q5U5X8"
}